{
  "gene": "UniProtKB:P78549",
  "gene_name": "Endonuclease III-like protein 1",
  "term_id": "GO:0000703",
  "gene_symbol": "NTHL1",
  "term_label": "oxidized pyrimidine nucleobase lesion DNA N-glycosylase activity"
}